cytolysis [GO:0019835] (biological process) Subtypes: cytolysis in another organism [GO:0051715] Sources: UniProtKB-KW:KW-0204 Also known as: lysis, autolysin activity, bacteriocin activity, bacteriolytic toxin activity, holin, lysin activity, necrosis Definition: The rupture of cell membranes and the loss of cytoplasm. Relationships: is a type of cellular process [GO:0009987] Regulation: regulated by regulation of cytolysis [GO:0042268]; negatively regulated by negative regulation of cytolysis [GO:0045918]; positively regulated by GO:0045919